{
  "term_label": "external side of plasma membrane",
  "gene_name": "C-type lectin domain family 4 member F",
  "gene": "UniProtKB:Q8N1N0",
  "gene_symbol": "CLEC4F",
  "term_id": "GO:0009897"
}